{
  "gene_name": "Perilipin-4",
  "term_label": "Unknown biological process",
  "gene_symbol": "PLIN4",
  "gene": "UniProtKB:Q96Q06",
  "term_id": "UNKNOWN:0002"
}